{
  "term_id": "GO:0016020",
  "gene": "UniProtKB:O75915",
  "gene_name": "PRA1 family protein 3",
  "gene_symbol": "ARL6IP5",
  "term_label": "membrane"
}